{
  "gene_symbol": "TIPRL",
  "term_label": "protein phosphatase activator activity",
  "gene_name": "TIP41-like protein",
  "term_id": "GO:0072542",
  "gene": "UniProtKB:O75663"
}